{
  "gene_name": "Probable threonine protease PRSS50",
  "gene_symbol": "PRSS50",
  "term_id": "GO:0008236",
  "term_label": "serine-type peptidase activity",
  "gene": "UniProtKB:Q9UI38"
}